{
  "term_label": "intracellular protein localization",
  "gene_name": "14-3-3 protein gamma",
  "term_id": "GO:0008104",
  "gene": "UniProtKB:P61981",
  "gene_symbol": "YWHAG"
}